{
  "term_id": "GO:0016324",
  "gene": "UniProtKB:Q2M3G4",
  "gene_name": "Protein Shroom1",
  "term_label": "apical plasma membrane",
  "gene_symbol": "SHROOM1"
}